potassium ion import across plasma membrane [GO:1990573] (biological process) Definition: The directed movement of potassium ions from outside of a cell, across the plasma membrane and into the cytosol. References: PMID:9139127 Also known as: potassium import, potassium ion import, potassium ion uptake Relationships: is a type of GO:0071805; is a type of inorganic cation import across plasma membrane [GO:0098659] Regulation: regulated by regulation of potassium ion import [GO:1903286]; RO_0002212 by negative regulation of potassium ion import across plasma membrane [GO:1903287]; RO_0002213 by positive regulation of potassium ion import across plasma membrane [GO:1903288]